negative regulation of tongue muscle cell differentiation [GO:2001036] (biological process) Sources: GOC:obol Relationships: is a type of negative regulation of skeletal muscle fiber differentiation [GO:1902810]; is_a regulation of tongue muscle cell differentiation [GO:2001035]; negatively regulates tongue muscle cell differentiation [GO:0035981] Definition: Any process that stops, prevents or reduces the frequency, rate or extent of tongue muscle cell differentiation.